chloroplast chromosome [GO:0042648] (cellular component) Definition: A circular DNA molecule containing chloroplast encoded genes. Sources: GOC:jl Relationships: is a type of plastid chromosome [GO:0009508]; is part of GO:0042644